{
  "term_label": "basolateral plasma membrane",
  "gene_name": "Electrogenic sodium bicarbonate cotransporter 1",
  "gene_symbol": "SLC4A4",
  "gene": "UniProtKB:Q9Y6R1",
  "term_id": "GO:0016323"
}